{
  "gene_name": "Putative uncharacterized protein FLJ35723",
  "term_label": "Unknown molecular function",
  "term_id": "UNKNOWN:0001",
  "gene_symbol": "Q8NA96",
  "gene": "UniProtKB:Q8NA96"
}